gonadotropin secretion [GO:0032274] (biological process) Subtypes: luteinizing hormone secretion [GO:0032275], follicle-stimulating hormone secretion [GO:0046884] Regulation: regulated by regulation of gonadotropin secretion [GO:0032276]; negatively regulated by negative regulation of gonadotropin secretion [GO:0032277]; positively regulated by positive regulation of gonadotropin secretion [GO:0032278] Sources: GOC:mah, ISBN:0721662544 Definition: The regulated release of a gonadotropin, any hormone that stimulates the gonads, especially follicle-stimulating hormone and luteinizing hormone. Relationships: is a type of endocrine hormone secretion [GO:0060986] Also known as: gonadotrophin secretion